{
  "term_id": "GO:0017157",
  "gene_name": "Ras-related protein Rab-37",
  "term_label": "regulation of exocytosis",
  "gene_symbol": "RAB37",
  "gene": "UniProtKB:Q96AX2"
}